{
  "term_id": "GO:0006338",
  "gene_symbol": "HMGB4",
  "term_label": "chromatin remodeling",
  "gene_name": "High mobility group protein B4",
  "gene": "UniProtKB:Q8WW32"
}